amino-terminal vacuolar sorting propeptide binding [GO:0009940] (molecular function) References: PMID:10871276 Sources: GOC:sm Definition: Binding to an amino terminal propeptide, which functions as a sorting signal to sort away the soluble vacuolar protein from Golgi to lytic vacuole via clathrin-coated vesicles. Relationships: is a type of vacuolar sorting signal binding [GO:0010209]